fibroblast growth factor receptor signaling pathway involved in orbitofrontal cortex development [GO:0035607] (biological process) Relationships: is a type of fibroblast growth factor receptor signaling pathway [GO:0008543]; is part of orbitofrontal cortex development [GO:0021769] Definition: The series of molecular signals generated as a consequence of a fibroblast growth factor-type receptor binding to one of its physiological ligands, which contributes to the progression of the orbitofrontal cortex over time from its initial formation until its mature state. Also known as: FGF receptor signaling pathway involved in orbitofrontal cortex development, FGFR signaling pathway involved in orbitofrontal cortex development, fibroblast growth factor receptor signalling pathway involved in orbitofrontal cortex development Sources: GOC:yaf